mitochondrial membrane fission [GO:0090149] (biological process) Definition: A process that is carried out at the cellular level which results in the separation of a single continuous mitochondrial membrane into two membranes and contributes to mitochondrial fission. Also known as: membrane fission involved in mitochondrial fission, mitochondrial membrane scission Relationships: is a type of membrane fission [GO:0090148]; is part of mitochondrial fission [GO:0000266] Sources: GOC:ascb_2009, GOC:dph, GOC:tb